{
  "gene": "UniProtKB:Q9Y3B3",
  "gene_symbol": "TMED7",
  "gene_name": "Transmembrane emp24 domain-containing protein 7",
  "term_label": "Golgi organization",
  "term_id": "GO:0007030"
}